{
  "term_id": "UNKNOWN:0002",
  "gene_symbol": "SLC5A10",
  "gene": "UniProtKB:A0PJK1",
  "gene_name": "Sodium_mannose cotransporter SLC5A10",
  "term_label": "Unknown biological process"
}